{
  "gene_name": "Protein CFAP20DC",
  "term_id": "UNKNOWN:0001",
  "gene_symbol": "CFAP20DC",
  "term_label": "Unknown molecular function",
  "gene": "UniProtKB:Q6ZVT6"
}